{
  "gene_symbol": "GPRC5C",
  "gene": "UniProtKB:Q9NQ84",
  "term_label": "plasma membrane",
  "gene_name": "G-protein coupled receptor family C group 5 member C",
  "term_id": "GO:0005886"
}